{
  "gene_symbol": "DDX18",
  "gene": "UniProtKB:Q9NVP1",
  "gene_name": "ATP-dependent RNA helicase DDX18",
  "term_id": "GO:0005730",
  "term_label": "nucleolus"
}